Set1C/COMPASS complex [GO:0048188] (cellular component) Also known as: COMPASS complex, Set1/COMPASS complex, Set1C Relationships: is a type of histone methyltransferase complex [GO:0035097] Definition: A conserved protein complex that catalyzes methylation of histone H3. In Saccharomyces the complex contains Shg1p, Sdc1p, Swd1p, Swd2p, Swd3p, Spp1p, Bre2p, and the trithorax-related Set1p; in mammals it contains the catalytic subunit (SETD1A or SETD1B), WDR5, WDR82, RBBP5, ASH2L/ASH2, CXXC1/CFP1, HCFC1 and DPY30. References: PMID:11687631, PMID:11742990, PMID:11805083, PMID:12488447, PMID:18508253, PMID:18838538